{
  "gene": "UniProtKB:P43088",
  "gene_symbol": "PTGFR",
  "gene_name": "Prostaglandin F2-alpha receptor",
  "term_label": "positive regulation of cytosolic calcium ion concentration",
  "term_id": "GO:0007204"
}